{
  "term_label": "sperm individualization",
  "gene": "UniProtKB:A0A1B0GUW6",
  "gene_symbol": "SPEM3",
  "term_id": "GO:0007291",
  "gene_name": "Uncharacterized protein SPEM3"
}